L-histidine catabolic process to 2-oxoglutarate [GO:0019558] (biological process) Definition: The chemical reactions and pathways resulting in the breakdown of L-histidine into other compounds, including 2-oxoglutarate. Sources: GOC:go_curators Also known as: histidine catabolic process to 2-oxoglutarate, histidine breakdown to 2-oxoglutarate, histidine catabolic process to 2-ketoglutarate, histidine catabolic process to alpha-ketoglutarate, histidine catabolic process to alpha-oxoglutarate, histidine catabolism to 2-ketoglutarate, histidine catabolism to alpha-ketoglutarate, histidine catabolism to alpha-oxoglutarate, histidine degradation to 2-oxoglutarate Relationships: is a type of 2-oxoglutarate metabolic process [GO:0006103]; is_a GO:0006548